{
  "term_id": "UNKNOWN:0002",
  "gene_name": "DnaJ homolog subfamily C member 5G",
  "gene": "UniProtKB:Q8N7S2",
  "term_label": "Unknown biological process",
  "gene_symbol": "DNAJC5G"
}